positive regulation of amniotic stem cell differentiation [GO:2000799] (biological process) Definition: Any process that activates or increases the frequency, rate or extent of amniotic stem cell differentiation. Relationships: is a type of positive regulation of mesenchymal stem cell differentiation [GO:2000741]; is a type of GO:2000797; positively regulates amniotic stem cell differentiation [GO:0097086] Sources: GOC:obol